{
  "gene": "UniProtKB:P53539",
  "gene_symbol": "FOSB",
  "term_id": "GO:0005634",
  "gene_name": "Protein FosB",
  "term_label": "nucleus"
}